{
  "gene_symbol": "NAE1",
  "gene": "UniProtKB:Q13564",
  "term_label": "Unknown molecular function",
  "term_id": "UNKNOWN:0001",
  "gene_name": "NEDD8-activating enzyme E1 regulatory subunit"
}